{
  "gene": "UniProtKB:Q8NH92",
  "term_label": "signal transduction",
  "term_id": "GO:0007165",
  "gene_name": "Olfactory receptor 1S1",
  "gene_symbol": "OR1S1"
}